{
  "term_label": "extracellular region",
  "gene": "UniProtKB:Q9NR71",
  "gene_symbol": "ASAH2",
  "term_id": "GO:0005576",
  "gene_name": "Neutral ceramidase"
}